phosphate ion binding [GO:0042301] (molecular function) Sources: GOC:jl Definition: Binding to a phosphate ion. Relationships: is a type of anion binding [GO:0043168]